{
  "term_label": "Unknown molecular function",
  "gene_name": "Putative POTE ankyrin domain family member M",
  "term_id": "UNKNOWN:0001",
  "gene": "UniProtKB:A6NI47",
  "gene_symbol": "POTEM"
}